sym-norspermidine synthase activity [GO:0050314] (molecular function) Also known as: S-adenosylmethioninamine:propane-1,3-diamine 3-aminopropyltransferase activity Relationships: is_a transferase activity, transferring alkyl or aryl (other than methyl) groups [GO:0016765] Definition: Catalysis of the reaction: 1,3-diaminopropane + S-adenosylmethioninamine = S-methyl-5'-thioadenosine + bis(3-aminopropyl)amine + H+. Sources: EC:2.5.1.23, RHEA:23244